{
  "gene": "UniProtKB:O00472",
  "gene_symbol": "ELL2",
  "term_id": "GO:0042795",
  "gene_name": "RNA polymerase II elongation factor ELL2",
  "term_label": "snRNA transcription by RNA polymerase II"
}